protein C-terminal carboxyl O-methyltransferase activity [GO:0003880] (molecular function) Also known as: C-terminal protein carboxyl methyltransferase activity Definition: Catalysis of the transfer of a methyl group to the oxygen atom of a carboxyl group at the C-terminal of a protein. Subtypes: protein C-terminal S-isoprenylcysteine carboxyl O-methyltransferase activity [GO:0004671], protein C-terminal leucine carboxyl O-methyltransferase activity [GO:0018423] Relationships: is a type of protein carboxyl O-methyltransferase activity [GO:0051998] References: PMID:8428937